{
  "term_label": "Unknown molecular function",
  "gene": "UniProtKB:Q2WGJ8",
  "term_id": "UNKNOWN:0001",
  "gene_name": "Cation channel sperm-associated auxiliary subunit TMEM249",
  "gene_symbol": "TMEM249"
}